{
  "gene_name": "Anomalous homeobox protein",
  "gene_symbol": "ANHX",
  "term_label": "regulation of transcription by RNA polymerase II",
  "term_id": "GO:0006357",
  "gene": "UniProtKB:E9PGG2"
}